{
  "gene_name": "Putative zinc finger protein 75C",
  "gene_symbol": "ZNF75CP",
  "term_label": "RNA polymerase II cis-regulatory region sequence-specific DNA binding",
  "term_id": "GO:0000978",
  "gene": "UniProtKB:Q92670"
}